tRNA-specific adenosine-34 deaminase complex [GO:0052718] (cellular component) References: PMID:17875641 Definition: A protein complex that possesses tRNA-specific adenosine-34 deaminase activity. In eukaryotes the complex is a heterodimer; the subunits are known as Tad2p and Tad3p in yeasts and Adat2 and Adat3 in human. Also known as: tRNA-A34 deaminase complex Relationships: is a type of GO:0140535; is a type of catalytic complex [GO:1902494]